[methionine synthase] reductase (NADPH) activity [GO:0030586] (molecular function) Definition: Catalysis of the reaction: [methionine synthase]-cob(II)alamin + NADPH + H+ + S-adenosyl methionine = [methionine synthase]-methylcob(I)alamin + S-adenosylhomocysteine + NADP+. Also known as: [methionine synthase]-cobalamin methyltransferase (cob(II)alamin reducing) activity, 5-methyltetrahydrofolate-homocysteine methyltransferase reductase, methionine synthase cob(II)alamin reductase (methylating) activity, methionine synthase reductase activity, methionine synthase-cobalamin methyltransferase (cob(II)alamin reducing), methionine synthase-methylcob(I)alamin,S-adenosylhomocysteine:NADP+ oxidoreductase activity Sources: RHEA:23908 Relationships: is_a GO:0016723